{
  "gene_name": "Endoplasmic reticulum membrane adapter protein XK",
  "term_id": "GO:0030674",
  "gene_symbol": "XK",
  "gene": "UniProtKB:P51811",
  "term_label": "protein-macromolecule adaptor activity"
}